{
  "term_id": "GO:0003735",
  "gene_symbol": "RPL24",
  "term_label": "structural constituent of ribosome",
  "gene": "UniProtKB:P83731",
  "gene_name": "Large ribosomal subunit protein eL24"
}